{
  "term_id": "GO:0006382",
  "term_label": "adenosine to inosine editing",
  "gene_name": "Double-stranded RNA-specific editase 1",
  "gene_symbol": "ADARB1",
  "gene": "UniProtKB:P78563"
}